maintenance of polarity of larval imaginal disc epithelium [GO:0042251] (biological process) Definition: The maintenance of an established polarized larval imaginal disc epithelium. Sources: GOC:jl Relationships: is a type of establishment or maintenance of polarity of larval imaginal disc epithelium [GO:0016336]